{
  "gene_name": "Transmembrane emp24 domain-containing protein 6",
  "term_label": "COPII-coated ER to Golgi transport vesicle",
  "gene_symbol": "TMED6",
  "gene": "UniProtKB:Q8WW62",
  "term_id": "GO:0030134"
}